{
  "term_id": "GO:0007155",
  "term_label": "cell adhesion",
  "gene": "UniProtKB:Q9NZG7",
  "gene_name": "Ninjurin-2",
  "gene_symbol": "NINJ2"
}